{
  "term_id": "GO:0019372",
  "gene": "UniProtKB:O15296",
  "term_label": "lipoxygenase pathway",
  "gene_name": "Polyunsaturated fatty acid lipoxygenase ALOX15B",
  "gene_symbol": "ALOX15B"
}